{
  "term_label": "regulation of intracellular signal transduction",
  "gene_name": "Protein phosphatase 1K, mitochondrial",
  "gene": "UniProtKB:Q8N3J5",
  "gene_symbol": "PPM1K",
  "term_id": "GO:1902531"
}